{
  "term_id": "GO:0086039",
  "gene": "UniProtKB:P16615",
  "term_label": "P-type calcium transporter activity involved in regulation of cardiac muscle cell membrane potential",
  "gene_symbol": "ATP2A2",
  "gene_name": "Sarcoplasmic_endoplasmic reticulum calcium ATPase 2"
}